cellular response to manganese ion [GO:0071287] (biological process) Definition: Any process that results in a change in state or activity of a cell (in terms of movement, secretion, enzyme production, gene expression, etc.) as a result of a manganese ion stimulus. Subtypes: GO:1990737 Also known as: cellular response to manganese Relationships: is a type of response to manganese ion [GO:0010042]; is a type of cellular response to metal ion [GO:0071248] Regulation: regulated by regulation of cellular response to manganese ion [GO:1905802]; negatively regulated by negative regulation of cellular response to manganese ion [GO:1905803]; positively regulated by positive regulation of cellular response to manganese ion [GO:1905804] Sources: GOC:mah